symbiont-mediated perturbation of host ubiquitin-like protein modification [GO:0039648] (biological process) Definition: A process by which a symbiont alters ubiquitin-like protein modification of target proteins of either host or symbiont proteins. This includes ubiquitination, SUMOylation, NEDDylation, and ISG15ylation. The ubiquitination status of a protein  affects whether it is targeted to the proteasome for degradation. The host is defined as the larger of the organisms involved in a symbiotic interaction. Relationships: is a type of GO:0044068 Also known as: modulation by symbiont of host protein ubiquitination, modulation of host ubiquitin pathway by virus, symbiont-mediated perturbation of host protein SUMOlyation, symbiont-mediated perturbation of host protein ubiquitination References: PMID:25166298, PMID:26483404, PMID:26712804